basic amino acid transmembrane transport [GO:1990822] (biological process) Sources: GOC:dph, GOC:vw Subtypes: basic amino acid transmembrane export from vacuole [GO:0034488], GO:0034490, L-histidine transmembrane export from vacuole [GO:0089708], L-arginine transmembrane transport [GO:1903826] Relationships: is a type of amino acid transmembrane transport [GO:0003333]; is a type of basic amino acid transport [GO:0015802] Definition: The directed movement of basic amino acids from one side of a membrane to the other.